{
  "term_label": "DNA-binding transcription factor activity, RNA polymerase II-specific",
  "gene": "UniProtKB:Q8IYN0",
  "gene_name": "Zinc finger protein 100",
  "gene_symbol": "ZNF100",
  "term_id": "GO:0000981"
}